{
  "gene": "UniProtKB:Q49AN0",
  "term_id": "GO:0003677",
  "gene_symbol": "CRY2",
  "term_label": "DNA binding",
  "gene_name": "Cryptochrome-2"
}